gluconate 2-dehydrogenase activity [GO:0008873] (molecular function) Definition: Catalysis of the reaction: D-gluconate + NADP+ = 2-dehydro-D-gluconate + NADPH + H+. Sources: EC:1.1.1.215 Also known as: 2-keto-D-gluconate reductase activity, 2-ketogluconate reductase activity Relationships: is_a GO:0008875